{
  "gene_symbol": "NDUFA11",
  "gene_name": "NADH dehydrogenase [ubiquinone] 1 alpha subcomplex subunit 11",
  "gene": "UniProtKB:Q86Y39",
  "term_id": "GO:0045271",
  "term_label": "respiratory chain complex I"
}